pigment metabolic process involved in pigmentation [GO:0043474] (biological process) Sources: GOC:dph, GOC:jl, GOC:tb Definition: The chemical reactions and pathways involving a pigment, any general or particular coloring matter in living organisms, resulting in the deposition or aggregation of pigment in an organism, tissue or cell. Subtypes: pigment metabolic process involved in developmental pigmentation [GO:0043324], pigment biosynthetic process involved in pigment accumulation [GO:0043477], ocellus pigment metabolic process [GO:0046158] Relationships: is_a GO:0042440; is part of GO:0043473 Also known as: pigment metabolic process during pigmentation, pigment metabolism during pigmentation